retinal cone cell development [GO:0046549] (biological process) Sources: ISBN:0198506732 Relationships: is a type of eye photoreceptor cell development [GO:0042462]; is part of retinal cone cell differentiation [GO:0042670] Definition: Development of a cone cell, one of the sensory cells in the eye that reacts to the presence of light. Cone cells contain the photopigment iodopsin or cyanopsin and are responsible for photopic (daylight) vision.